{
  "term_label": "Unknown biological process",
  "gene": "UniProtKB:Q8N0Y3",
  "gene_name": "Olfactory receptor 4N4",
  "term_id": "UNKNOWN:0002",
  "gene_symbol": "OR4N4"
}